{
  "gene_symbol": "TSC22D4",
  "term_label": "Unknown cellular component",
  "gene": "UniProtKB:Q9Y3Q8",
  "gene_name": "TSC22 domain family protein 4",
  "term_id": "UNKNOWN:0003"
}